{
  "term_label": "cell-cell junction assembly",
  "term_id": "GO:0007043",
  "gene_symbol": "CDH3",
  "gene_name": "Cadherin-3",
  "gene": "UniProtKB:P22223"
}